aggresome [GO:0016235] (cellular component) Definition: An inclusion body formed by dynein-dependent retrograde transport of an aggregated protein on microtubules. References: PMID:11121744 Relationships: is a type of inclusion body [GO:0016234]